{
  "term_label": "Unknown cellular component",
  "term_id": "UNKNOWN:0003",
  "gene_name": "Retinol dehydrogenase 12",
  "gene": "UniProtKB:Q96NR8",
  "gene_symbol": "RDH12"
}